{
  "term_label": "mitotic cell cycle",
  "gene": "UniProtKB:Q9BVA1",
  "gene_name": "Tubulin beta-2B chain",
  "term_id": "GO:0000278",
  "gene_symbol": "TUBB2B"
}